{
  "gene_name": "Protein zwilch homolog",
  "term_id": "GO:1990423",
  "term_label": "RZZ complex",
  "gene_symbol": "ZWILCH",
  "gene": "UniProtKB:Q9H900"
}